{
  "gene_symbol": "ELMOD1",
  "term_label": "cilium assembly",
  "gene_name": "ELMO domain-containing protein 1",
  "gene": "UniProtKB:Q8N336",
  "term_id": "GO:0060271"
}